{
  "gene": "UniProtKB:Q9UHC6",
  "gene_name": "Contactin-associated protein-like 2",
  "term_id": "GO:0005886",
  "term_label": "plasma membrane",
  "gene_symbol": "CNTNAP2"
}